positive regulation of leaf senescence [GO:1900057] (biological process) Definition: Any process that activates or increases the frequency, rate or extent of leaf senescence. Also known as: activation of leaf senescence, up regulation of leaf senescence, up-regulation of leaf senescence, upregulation of leaf senescence Sources: GOC:TermGenie Relationships: is a type of positive regulation of developmental process [GO:0051094]; is a type of regulation of leaf senescence [GO:1900055]; positively regulates leaf senescence [GO:0010150]